{
  "gene_symbol": "NDP",
  "gene_name": "Norrin",
  "term_label": "positive regulation of DNA-templated transcription",
  "gene": "UniProtKB:Q00604",
  "term_id": "GO:0045893"
}